cyanidin 3-O-glucoside biosynthetic process [GO:0033485] (biological process) Sources: GOC:mah, MetaCyc:PWY-5125 Definition: The chemical reactions and pathways resulting in the formation of cyanidin 3-O-glucoside, a basic anthocyanin responsible for red to magenta coloration of flowers and fruits. Relationships: is_a flavonoid biosynthetic process [GO:0009813]; is a type of cyanidin 3-O-glucoside metabolic process [GO:1901038]; is a type of beta-glucoside biosynthetic process [GO:1901806] Also known as: cyanidin 3-O-glucoside anabolism, cyanidin 3-O-glucoside biosynthesis, cyanidin 3-O-glucoside formation, cyanidin 3-O-glucoside synthesis